{
  "term_label": "axonogenesis",
  "gene_symbol": "SLITRK2",
  "gene": "UniProtKB:Q9H156",
  "term_id": "GO:0007409",
  "gene_name": "SLIT and NTRK-like protein 2"
}